arachidonate transmembrane transporter activity [GO:1903962] (molecular function) Also known as: arachidonate transporter activity, arachidonic acid transporter activity Definition: Enables the transfer of arachidonate from one side of a membrane to the other. Relationships: is a type of long-chain fatty acid transmembrane transporter activity [GO:0005324]; is part of arachidonate transport [GO:1903963] Note: An example of this is S100A9 in human (P06702) in PMID:15642721 (inferred from direct assay). References: PMID:15642721 Sources: GOC:TermGenie, GOC:bhm, GO_REF:0000066